{
  "term_label": "inner dynein arm",
  "term_id": "GO:0036156",
  "gene_symbol": "DNAI3",
  "gene": "UniProtKB:Q8IWG1",
  "gene_name": "Dynein axonemal intermediate chain 3"
}